{
  "term_id": "GO:0045930",
  "gene_symbol": "BRINP1",
  "term_label": "negative regulation of mitotic cell cycle",
  "gene_name": "BMP_retinoic acid-inducible neural-specific protein 1",
  "gene": "UniProtKB:O60477"
}